{
  "gene_symbol": "SORBS3",
  "term_id": "GO:0030055",
  "term_label": "cell-substrate junction",
  "gene_name": "Vinexin",
  "gene": "UniProtKB:O60504"
}